{
  "term_id": "GO:0005925",
  "gene_name": "Integrin beta-4",
  "gene": "UniProtKB:P16144",
  "term_label": "focal adhesion",
  "gene_symbol": "ITGB4"
}